4-hydroxybenzoate 3-monooxygenase activity [GO:0018659] (molecular function) Definition: Catalysis of the reaction: 4-hydroxybenzoate + NADPH + H+ + O2 = protocatechuate + NADP+ + H2O. Also known as: 4-hydroxybenzoate 3-hydroxylase activity, p-hydroxybenzoate hydroxylase activity, p-hydroxybenzoic acid hydroxylase activity, para-hydroxybenzoate hydroxylase activity, 4-hydroxybenzoate monooxygenase activity, 4-hydroxybenzoate,NADPH:oxygen oxidoreductase (3-hydroxylating), p-hydroxybenzoate hydrolyase activity, p-hydroxybenzoate-3-hydroxylase activity, p-hydroxybenzoic acid hydrolase activity, p-hydroxybenzoic hydroxylase activity Sources: EC:1.14.13.2 Relationships: is a type of oxidoreductase activity, acting on paired donors, with incorporation or reduction of molecular oxygen, NAD(P)H as one donor, and incorporation of one atom of oxygen [GO:0016709]